{
  "term_id": "GO:0015279",
  "gene_name": "Protein orai-3",
  "gene_symbol": "ORAI3",
  "gene": "UniProtKB:Q9BRQ5",
  "term_label": "store-operated calcium channel activity"
}